{
  "gene_name": "Interleukin-1 receptor-associated kinase 1-binding protein 1",
  "gene": "UniProtKB:Q5VVH5",
  "gene_symbol": "IRAK1BP1",
  "term_id": "UNKNOWN:0002",
  "term_label": "Unknown biological process"
}